{
  "gene_symbol": "SI",
  "term_id": "UNKNOWN:0003",
  "gene_name": "Sucrase-isomaltase, intestinal",
  "term_label": "Unknown cellular component",
  "gene": "UniProtKB:P14410"
}